{
  "term_id": "GO:0005737",
  "gene_symbol": "TRIM75",
  "gene_name": "Tripartite motif-containing protein 75",
  "gene": "UniProtKB:A6NK02",
  "term_label": "cytoplasm"
}